{
  "term_label": "Unknown biological process",
  "term_id": "UNKNOWN:0002",
  "gene_name": "Calmodulin-lysine N-methyltransferase",
  "gene": "UniProtKB:Q7Z624",
  "gene_symbol": "CAMKMT"
}